{
  "gene": "UniProtKB:Q9Y2W7",
  "gene_name": "Calsenilin",
  "term_label": "voltage-gated potassium channel complex",
  "term_id": "GO:0008076",
  "gene_symbol": "KCNIP3"
}